{
  "term_label": "ubiquitin protein ligase activity",
  "term_id": "GO:0061630",
  "gene_symbol": "TRIM4",
  "gene": "UniProtKB:Q9C037",
  "gene_name": "E3 ubiquitin-protein ligase TRIM4"
}